{
  "term_id": "GO:0006955",
  "term_label": "immune response",
  "gene": "UniProtKB:P09326",
  "gene_symbol": "CD48",
  "gene_name": "CD48 antigen"
}